chemical synaptic transmission, postsynaptic [GO:0099565] (biological process) Relationships: is a type of cell surface receptor signaling pathway [GO:0007166]; is a type of nervous system process [GO:0050877]; is part of GO:0007268; occurs in postsynapse [GO:0098794] Also known as: postsynaptic process involved in chemical synaptic transmission Definition: The part of synaptic transmission occurring in the post-synapse: a signal transduction pathway consisting of neurotransmitter receptor activation and its effects on postsynaptic membrane potential and the ionic composition of the postsynaptic cytosol. Sources: GOC:dos